{
  "gene": "UniProtKB:P58499",
  "gene_symbol": "FAM3B",
  "gene_name": "Protein FAM3B",
  "term_id": "GO:0005615",
  "term_label": "extracellular space"
}